synaptobrevin 2-SNAP-25-syntaxin-1a-complexin II complex [GO:0070033] (cellular component) Definition: A SNARE complex that contains synaptobrevin 2 (VAMP2), SNAP-25, syntaxin 1a, and complexin II (or orthologs thereof). References: PMID:7553862 Also known as: SNARE complex (Vamp2, Snap25, Stx1a, Cplx2), Vamp2-Snap25-Stx1a-Cplx2 complex Relationships: is a type of SNARE complex [GO:0031201]